{
  "gene_name": "17-beta-hydroxysteroid dehydrogenase type 6",
  "term_id": "GO:0004745",
  "gene_symbol": "HSD17B6",
  "term_label": "all-trans-retinol dehydrogenase (NAD+) activity",
  "gene": "UniProtKB:O14756"
}